{
  "gene_name": "Sarcosine dehydrogenase, mitochondrial",
  "gene": "UniProtKB:Q9UL12",
  "term_id": "GO:0005739",
  "term_label": "mitochondrion",
  "gene_symbol": "SARDH"
}